{
  "gene_symbol": "PABPC4",
  "term_label": "mRNA 3'-UTR binding",
  "gene_name": "Polyadenylate-binding protein 4",
  "gene": "UniProtKB:Q13310",
  "term_id": "GO:0003730"
}